{
  "gene_name": "Ankyrin repeat domain-containing protein 46",
  "gene_symbol": "ANKRD46",
  "gene": "UniProtKB:Q86W74",
  "term_id": "UNKNOWN:0001",
  "term_label": "Unknown molecular function"
}